{
  "gene": "UniProtKB:Q9Y6C2",
  "term_id": "UNKNOWN:0002",
  "term_label": "Unknown biological process",
  "gene_name": "EMILIN-1",
  "gene_symbol": "EMILIN1"
}